extracellular matrix organization [GO:0030198] (biological process) Regulation: regulated by GO:1903053; negatively regulated by negative regulation of extracellular matrix organization [GO:1903054]; positively regulated by GO:1903055 Definition: A process that is carried out at the cellular level which results in the assembly, arrangement of constituent parts, or disassembly of an extracellular matrix. Sources: GOC:mah Also known as: extracellular matrix organisation, extracellular matrix organization and biogenesis Relationships: is a type of extracellular structure organization [GO:0043062]; is a type of external encapsulating structure organization [GO:0045229] Subtypes: cellulose microfibril organization [GO:0010215], GO:0021820, extracellular matrix disassembly [GO:0022617], collagen fibril organization [GO:0030199], glomerular basement membrane development [GO:0032836], extracellular matrix organization involved in endocardium development [GO:0061148], basement membrane organization [GO:0071711], extracellular matrix assembly [GO:0085029], biofilm matrix organization [GO:0098784]